{
  "gene": "UniProtKB:Q9H1X1",
  "gene_name": "Radial spoke head protein 9 homolog",
  "gene_symbol": "RSPH9",
  "term_id": "UNKNOWN:0001",
  "term_label": "Unknown molecular function"
}